{
  "gene_name": "G-protein coupled receptor family C group 5 member B",
  "gene": "UniProtKB:Q9NZH0",
  "gene_symbol": "GPRC5B",
  "term_id": "GO:0030295",
  "term_label": "protein kinase activator activity"
}